{
  "gene_name": "Immunoglobulin lambda joining 4 (non-functional) (Fragment)",
  "term_id": "UNKNOWN:0003",
  "term_label": "Unknown cellular component",
  "gene_symbol": "IGLJ4",
  "gene": "UniProtKB:A0A0A0MTA1"
}